{
  "gene_name": "Fibronectin type 3 and ankyrin repeat domains protein 1",
  "term_id": "UNKNOWN:0001",
  "gene_symbol": "FANK1",
  "gene": "UniProtKB:Q8TC84",
  "term_label": "Unknown molecular function"
}